meiotic DNA double-strand break formation involved in reciprocal meiotic recombination [GO:0010780] (biological process) Sources: GOC:dph, GOC:tb Relationships: is a type of meiotic DNA double-strand break formation [GO:0042138]; is part of reciprocal meiotic recombination [GO:0007131] Definition: The cell cycle process in which double-strand breaks are generated at defined hotspots throughout the genome during meiosis I resulting in meiotic recombination. Meiotic recombination is the cell cycle process in which double strand breaks are formed and repaired through a double Holliday junction intermediate. Regulation: RO_0002211 by regulation of meiotic DNA double-strand break formation involved in reciprocal meiotic recombination [GO:1905261]; negatively regulated by negative regulation of meiotic DNA double-strand break formation involved in reciprocal meiotic recombination [GO:1905262]; positively regulated by positive regulation of meiotic DNA double-strand break formation involved in reciprocal meiotic recombination [GO:1905263]